{
  "gene_symbol": "TSPAN11",
  "term_id": "GO:0005886",
  "term_label": "plasma membrane",
  "gene_name": "Tetraspanin-11",
  "gene": "UniProtKB:A1L157"
}